{
  "term_label": "macroautophagy",
  "term_id": "GO:0016236",
  "gene_name": "Etoposide-induced protein 2.4 homolog",
  "gene": "UniProtKB:O14681",
  "gene_symbol": "EI24"
}